{
  "term_id": "GO:0032052",
  "term_label": "bile acid binding",
  "gene": "UniProtKB:P42330",
  "gene_name": "Aldo-keto reductase family 1 member C3",
  "gene_symbol": "AKR1C3"
}